{
  "term_id": "UNKNOWN:0003",
  "gene_symbol": "TMEM81",
  "term_label": "Unknown cellular component",
  "gene": "UniProtKB:Q6P7N7",
  "gene_name": "Transmembrane protein 81"
}